negative regulation of mini excitatory postsynaptic potential [GO:0061886] (biological process) Definition: Any process that decreases the frequency, rate or extent of mini excitatory postsynaptic potential. Mini excitatory postsynaptic potential is a process that leads to a temporary increase in postsynaptic potential due to the flow of positively charged ions into the postsynaptic cell, induced by the spontaneous release of a single vesicle of an excitatory neurotransmitter into the synapse. References: PMID:20395454 Sources: GOC:aruk, GOC:bc Relationships: is a type of regulation of mini excitatory postsynaptic potential [GO:0061884]; is_a negative regulation of excitatory postsynaptic potential [GO:0090394]; RO_0002212 mini excitatory postsynaptic potential [GO:0098816]